regulation of shade avoidance [GO:1902446] (biological process) Definition: Any process that modulates the frequency, rate or extent of shade avoidance. References: PMID:23763263 Sources: GOC:TermGenie Subtypes: negative regulation of shade avoidance [GO:1902447], positive regulation of shade avoidance [GO:1902448] Relationships: is a type of regulation of response to red or far red light [GO:2000030]; regulates shade avoidance [GO:0009641]